{
  "gene": "UniProtKB:Q9Y5E7",
  "term_id": "GO:0007155",
  "term_label": "cell adhesion",
  "gene_name": "Protocadherin beta-2",
  "gene_symbol": "PCDHB2"
}